cellular response to phosphatidylethanolamine [GO:1905712] (biological process) References: PMID:1657995 Sources: GOC:TermGenie, GO_REF:0000071 Relationships: is a type of cellular response to lipid [GO:0071396]; is a type of GO:1901701; is a type of response to phosphatidylethanolamine [GO:1905711] Also known as: cellular response to PE, cellular response to PtdEtn, cellular response to phosphatidyl(amino)ethanols, cellular response to phosphatidylethanolamines Definition: Any process that results in a change in state or activity of a cell (in terms of movement, secretion, enzyme production, gene expression, etc.) as a result of a phosphatidylethanolamine stimulus.